{
  "term_label": "regulation of cytosolic calcium ion concentration",
  "gene": "UniProtKB:P48995",
  "term_id": "GO:0051480",
  "gene_symbol": "TRPC1",
  "gene_name": "Short transient receptor potential channel 1"
}